nucleoplasmic reticulum [GO:0044195] (cellular component) Definition: Long, dynamic tubular channels, formed by invagination of the nuclear envelope, that extend deep into the nucleoplasm. The channels have an underlying lamina and are implicated in functioning in signaling and transport. Relationships: is a type of cellular anatomical structure [GO:0110165]; is part of GO:0005635 Also known as: nuclear channels References: PMID:17959832, PMID:9024685 Sources: GOC:jl